{
  "term_label": "aminoacyl-tRNA synthetase multienzyme complex",
  "gene_name": "Methionine--tRNA ligase, cytoplasmic",
  "gene_symbol": "MARS1",
  "term_id": "GO:0017101",
  "gene": "UniProtKB:P56192"
}